RNA splicing, via transesterification reactions with guanosine as nucleophile [GO:0000376] (BP) References: PMID:11377794 Sources: GOC:krc Relationships: is a type of GO:0000375 Subtypes: GO:0000372 Definition: Splicing of RNA via a series of two transesterification reactions with exogenous guanosine as the initiating nucleophile.